{
  "gene_name": "CEP295 N-terminal-like protein",
  "gene_symbol": "CEP295NL",
  "term_id": "GO:0005813",
  "term_label": "centrosome",
  "gene": "UniProtKB:Q96MC4"
}